{
  "gene_symbol": "RAB6A",
  "gene": "UniProtKB:P20340",
  "gene_name": "Ras-related protein Rab-6A",
  "term_id": "GO:0006886",
  "term_label": "intracellular protein transport"
}